{
  "gene_symbol": "KIAA1614",
  "term_label": "centrosome cycle",
  "gene": "UniProtKB:Q5VZ46",
  "gene_name": "Uncharacterized protein KIAA1614",
  "term_id": "GO:0007098"
}